spinal cord association neuron differentiation [GO:0021527] (biological process) References: PMID:11262869 Sources: GOC:cls, GOC:dgh, GOC:dph, GOC:jid, GO_REF:0000021 Regulation: regulated by regulation of spinal cord association neuron differentiation [GO:1902829]; negatively regulated by GO:1902830; positively regulated by positive regulation of spinal cord association neuron differentiation [GO:1902831] Relationships: is a type of GO:0021515; is a type of central nervous system neuron differentiation [GO:0021953]; is part of GO:0021516 Definition: The process in which neuroepithelial cells in the neural tube acquire specialized structural and/or functional features of association neurons. Association neurons are cells located in the dorsal portion of the spinal cord that integrate sensory input. Differentiation includes the processes involved in commitment of a cell to a specific fate. Also known as: spinal cord dorsal interneuron differentiation